MHC class II protein complex [GO:0042613] (cellular component) Relationships: is a type of GO:0042611 Definition: A transmembrane protein complex composed of an MHC class II alpha and MHC class II beta chain, and with or without a bound peptide or polysaccharide antigen. References: PMID:15928678 Sources: GOC:add, GOC:jl, ISBN:0120781859